{
  "gene": "UniProtKB:Q8N4P2",
  "gene_name": "Intraflagellar transport protein 70B",
  "gene_symbol": "IFT70B",
  "term_label": "intraciliary transport particle B",
  "term_id": "GO:0030992"
}